chromatophore ribulose bisphosphate carboxylase complex [GO:0048494] (cellular component) Sources: GOC:mlg, GOC:mtg_sensu Also known as: RubisCO complex Subtypes: plasma membrane-derived thylakoid ribulose bisphosphate carboxylase complex [GO:0048493] Relationships: is a type of GO:0048492; is part of plasma membrane-derived chromatophore [GO:0042716] Definition: A complex, located in the chromatophore, containing either both large and small subunits or just small subunits which carries out the activity of producing 3-phosphoglycerate from carbon dioxide and ribulose-1,5-bisphosphate.